{
  "term_label": "Unknown cellular component",
  "term_id": "UNKNOWN:0003",
  "gene_symbol": "SMYD5",
  "gene_name": "Histone-lysine N-trimethyltransferase SMYD5",
  "gene": "UniProtKB:Q6GMV2"
}